negative regulation of inositol trisphosphate biosynthetic process [GO:0032961] (biological process) Sources: GOC:mah Definition: Any process that stops, prevents, or reduces the frequency, rate or extent of the chemical reactions and pathways resulting in the formation of inositol trisphosphate. Relationships: is a type of negative regulation of inositol phosphate biosynthetic process [GO:0010920]; is a type of GO:0032960; negatively regulates GO:0032959 Also known as: negative regulation of IP3 biosynthesis, negative regulation of IP3 biosynthetic process, negative regulation of inositol trisphosphate anabolism, negative regulation of inositol trisphosphate biosynthesis, negative regulation of inositol trisphosphate formation, negative regulation of inositol trisphosphate synthesis, negative regulation of myo-inositol trisphosphate biosynthesis, negative regulation of myo-inositol trisphosphate biosynthetic process